{
  "term_id": "GO:0007166",
  "gene_name": "T cell receptor beta variable 7-9",
  "gene": "UniProtKB:P04435",
  "term_label": "cell surface receptor signaling pathway",
  "gene_symbol": "TRBV7-9"
}